{
  "gene_name": "Coiled-coil domain-containing protein 40",
  "gene": "UniProtKB:Q4G0X9",
  "term_label": "Unknown molecular function",
  "gene_symbol": "CCDC40",
  "term_id": "UNKNOWN:0001"
}